{
  "gene": "UniProtKB:O00391",
  "term_label": "protein folding",
  "gene_name": "Sulfhydryl oxidase 1",
  "gene_symbol": "QSOX1",
  "term_id": "GO:0006457"
}